{
  "gene_symbol": "RIMS2",
  "term_id": "GO:0098882",
  "gene_name": "Regulating synaptic membrane exocytosis protein 2",
  "term_label": "structural constituent of presynaptic active zone",
  "gene": "UniProtKB:Q9UQ26"
}